{
  "term_id": "GO:0004715",
  "gene_name": "Tyrosine-protein kinase CSK",
  "term_label": "non-membrane spanning protein tyrosine kinase activity",
  "gene": "UniProtKB:P41240",
  "gene_symbol": "CSK"
}